regulation of glucomannan catabolic process [GO:2000898] (biological process) Also known as: regulation of glucomannan catabolism Sources: GOC:mengo_curators Relationships: is a type of regulation of polysaccharide metabolic process [GO:0032881]; is_a regulation of carbohydrate catabolic process [GO:0043470]; RO_0002211 GO:2000884 Definition: Any process that modulates the frequency, rate or extent of glucomannan catabolic process. Subtypes: negative regulation of glucomannan catabolic process [GO:2000907], positive regulation of glucomannan catabolic process [GO:2000908]